lateral mesoderm formation [GO:0048370] (biological process) Also known as: lateral plate mesoderm biosynthesis, lateral plate mesoderm formation Sources: GOC:jid Relationships: is_a GO:0001707; is part of lateral mesoderm morphogenesis [GO:0048369] Definition: The process that gives rise to the lateral mesoderm. This process pertains to the initial formation of the structure from unspecified parts.